D-glycero-D-manno-heptose 7-phosphate biosynthetic process [GO:2001061] (biological process) Definition: The chemical reactions and pathways resulting in the formation of a D-glycero-D-manno-heptose 7-phosphate. Sources: GOC:mengo_curators Also known as: D-glycero-D-manno-heptose 7-phosphate biosynthesis Relationships: is_a organophosphate biosynthetic process [GO:0090407]; is a type of carbohydrate derivative biosynthetic process [GO:1901137]; is_a GO:2001060